{
  "term_label": "Unknown biological process",
  "gene": "UniProtKB:P0DW85",
  "gene_name": "Histone H2A.N",
  "gene_symbol": "H2BN1",
  "term_id": "UNKNOWN:0002"
}